negative regulation of emericellamide biosynthetic process [GO:1900659] (biological process) Subtypes: negative regulation of emericellamide A biosynthetic process [GO:1900662] Definition: Any process that stops, prevents or reduces the frequency, rate or extent of emericellamide biosynthetic process. Sources: GOC:TermGenie, GOC:di Relationships: is a type of negative regulation of amide metabolic process [GO:0034249]; is a type of GO:0051055; is a type of negative regulation of small molecule metabolic process [GO:0062014]; is a type of GO:1900377; is_a regulation of emericellamide biosynthetic process [GO:1900658]; negatively regulates GO:1900557 Also known as: down regulation of emericellamide anabolism, down regulation of emericellamide biosynthesis, down regulation of emericellamide biosynthetic process, down regulation of emericellamide formation, down regulation of emericellamide synthesis, down-regulation of emericellamide anabolism, down-regulation of emericellamide biosynthesis, down-regulation of emericellamide biosynthetic process, down-regulation of emericellamide formation, down-regulation of emericellamide synthesis, downregulation of emericellamide anabolism, downregulation of emericellamide biosynthesis, downregulation of emericellamide biosynthetic process, downregulation of emericellamide formation, downregulation of emericellamide synthesis, inhibition of emericellamide anabolism, inhibition of emericellamide biosynthesis, inhibition of emericellamide formation, inhibition of emericellamide synthesis, negative regulation of emericellamide anabolism, negative regulation of emericellamide biosynthesis, negative regulation of emericellamide formation, negative regulation of emericellamide synthesis, inhibition of emericellamide biosynthetic process